{
  "gene": "UniProtKB:Q86U42",
  "gene_symbol": "PABPN1",
  "term_id": "GO:0008143",
  "gene_name": "Polyadenylate-binding protein 2",
  "term_label": "poly(A) binding"
}